{
  "gene_symbol": "KCNAB3",
  "gene": "UniProtKB:O43448",
  "gene_name": "Voltage-gated potassium channel subunit beta-3",
  "term_id": "GO:1901379",
  "term_label": "regulation of potassium ion transmembrane transport"
}